renal system vasculature development [GO:0061437] (biological process) Relationships: is a type of vasculature development [GO:0001944]; is part of renal system development [GO:0072001] References: PMID:11891195 Sources: GOC:dph, GOC:mtg_kidney_jan10 Subtypes: GO:0061440 Definition: The process whose specific outcome is the progression of vasculature of the renal system over time, from its formation to the mature structure.